{
  "gene_name": "Nicotinamide riboside kinase 1",
  "term_id": "UNKNOWN:0002",
  "gene": "UniProtKB:Q9NWW6",
  "term_label": "Unknown biological process",
  "gene_symbol": "NMRK1"
}